{
  "term_label": "Unknown cellular component",
  "gene_name": "Endogenous retrovirus group K member 13-1 Env polyprotein",
  "gene": "UniProtKB:Q9NX77",
  "gene_symbol": "ERVK13-1",
  "term_id": "UNKNOWN:0003"
}